cerebellar granular layer maturation [GO:0021686] (BP) Sources: GOC:cls, GOC:dgh, GOC:dph, GOC:jid, GO_REF:0000021 Definition: A developmental process, independent of morphogenetic (shape) change, that is required for the cerebellar granular layer to attain its fully functional state. The granular layer is the innermost layer of the cerebellar cortex. This layer contains densely packed small neurons, mostly granule cells. Some Golgi cells are found at the outer border. Granule neurons send parallel fibers to the upper molecular layer, where they synapse with Purkinje cell dendrites. Mossy fibers from the pontine nuclei in the white matter synapse with granule cell axons, Golgi cell axons and unipolar brush interneuron axons at cerebellar glomeruli in the granule cell layer. Relationships: is a type of anatomical structure maturation [GO:0071695]; is part of cerebellar granular layer development [GO:0021681]; is part of cerebellar cortex maturation [GO:0021699]